cell wall glycoprotein biosynthetic process [GO:0031506] (biological process) Definition: The chemical reactions and pathways resulting in the formation of cell wall glycoproteins, any cell wall protein that contains covalently bound sugar residues. Sources: GOC:mah Also known as: cell wall glycoprotein anabolism, cell wall glycoprotein biosynthesis, cell wall glycoprotein formation, cell wall glycoprotein synthesis Relationships: is a type of glycoprotein biosynthetic process [GO:0009101]; is a type of cell wall macromolecule biosynthetic process [GO:0044038] Subtypes: cell wall mannoprotein biosynthetic process [GO:0000032]